adhesion between unicellular organisms [GO:0098610] (biological process) Sources: GOC:dos Also known as: multi-organismal cell-cell adhesion, adhesion between unicellular organisms via cell-wall interaction Subtypes: GO:0000128, GO:0000761 Definition: The attachment of two unicellular organisms to each other. Relationships: is a type of cell-cell adhesion [GO:0098609]